{
  "term_id": "UNKNOWN:0002",
  "gene": "UniProtKB:Q6W349",
  "gene_symbol": "LINC00575",
  "gene_name": "Putative uncharacterized protein encoded by LINC00575",
  "term_label": "Unknown biological process"
}